{
  "term_label": "Unknown biological process",
  "gene_name": "Uncharacterized protein C16orf46",
  "gene": "UniProtKB:Q6P387",
  "gene_symbol": "C16orf46",
  "term_id": "UNKNOWN:0002"
}